chondroitin 2-sulfotransferase activity [GO:0034482] (molecular function) References: PMID:17227754 Relationships: is a type of GO:0034481 Definition: Catalysis of the reaction: 3'-phosphoadenosine 5'-phosphosulfate + chondroitin = adenosine 3',5'-bisphosphate + chondroitin 2'-O-sulfate. Results in sulfation of glucuronic acid and iduronic acid residues. Also known as: chondroitin 2-O-sulfotransferase activity, chondroitin 2-O-sulphotransferase activity